{
  "term_label": "postsynaptic density membrane",
  "gene_symbol": "DLG4",
  "term_id": "GO:0098839",
  "gene_name": "Disks large homolog 4",
  "gene": "UniProtKB:P78352"
}